{
  "term_label": "lipopolysaccharide immune receptor activity",
  "gene": "UniProtKB:O00206",
  "term_id": "GO:0001875",
  "gene_name": "Toll-like receptor 4",
  "gene_symbol": "TLR4"
}